{
  "gene_symbol": "CHML",
  "gene": "UniProtKB:P26374",
  "gene_name": "Rab proteins geranylgeranyltransferase component A 2",
  "term_label": "Unknown molecular function",
  "term_id": "UNKNOWN:0001"
}